{
  "gene_symbol": "C17orf58",
  "gene_name": "UPF0450 protein C17orf58",
  "term_label": "Unknown molecular function",
  "term_id": "UNKNOWN:0001",
  "gene": "UniProtKB:Q2M2W7"
}